exodeoxyribonuclease VII complex [GO:0009318] (cellular component) Relationships: is a type of intracellular protein-containing complex [GO:0140535]; is a type of catalytic complex [GO:1902494] References: PMID:6284744 Definition: An enzyme complex that catalyzes exonucleolytic cleavage in either 5' to 3' or 3' to 5' direction to yield nucleoside 5'-phosphates; it prefers single-stranded DNA.